regulation of intrinsic apoptotic signaling pathway in response to DNA damage [GO:1902229] (biological process) References: PMID:15314165 Sources: GOC:BHF, GOC:TermGenie, GOC:mtg_apoptosis, GOC:rl Also known as: regulation of DNA damage response, signal transduction resulting in induction of apoptosis Subtypes: GO:1902165, negative regulation of intrinsic apoptotic signaling pathway in response to DNA damage [GO:1902230], positive regulation of intrinsic apoptotic signaling pathway in response to DNA damage [GO:1902231] Relationships: is a type of GO:0080135; is a type of GO:2001242; regulates intrinsic apoptotic signaling pathway in response to DNA damage [GO:0008630] Definition: Any process that modulates the frequency, rate or extent of intrinsic apoptotic signaling pathway in response to DNA damage.